{
  "term_id": "GO:0042383",
  "gene": "UniProtKB:Q6ZMU5",
  "gene_symbol": "TRIM72",
  "term_label": "sarcolemma",
  "gene_name": "Tripartite motif-containing protein 72"
}